{
  "gene": "UniProtKB:Q14568",
  "gene_name": "Heat shock protein HSP 90-alpha A2",
  "gene_symbol": "HSP90AA2P",
  "term_id": "GO:0048471",
  "term_label": "perinuclear region of cytoplasm"
}